{
  "gene_name": "Allergin-1",
  "term_label": "immune response",
  "gene": "UniProtKB:Q7Z6M3",
  "term_id": "GO:0006955",
  "gene_symbol": "MILR1"
}